{
  "gene_name": "Serine_threonine-protein kinase MRCK alpha",
  "gene_symbol": "CDC42BPA",
  "gene": "UniProtKB:Q5VT25",
  "term_id": "GO:0005737",
  "term_label": "cytoplasm"
}